anterior lateral line nerve development [GO:0048909] (biological process) Sources: GOC:cls, GOC:dgh, GOC:dph, GOC:jid, GO_REF:0000021 Definition: The process whose specific outcome is the progression of the anterior lateral line nerve over time, form its formation to the mature structure. The anterior lateral line nerve contains efferent axons that innervate hair cells of the ALL and afferent axons that project to an octavolateralis column in the hindbrain. The octavolateralis column consists of the medial octavolateralis nucleus (MON), the caudal octavolateralis nucleus, and the magnocellular nucleus. Also known as: ALLN development, nALL development, rostral lateral line nerve development Relationships: is a type of lateral line nerve development [GO:0048892]; is part of anterior lateral line system development [GO:0048898]